{
  "gene_symbol": "NGF",
  "gene": "UniProtKB:P01138",
  "term_label": "cell surface receptor protein tyrosine kinase signaling pathway",
  "gene_name": "Beta-nerve growth factor",
  "term_id": "GO:0007169"
}